{
  "term_label": "centrosome localization",
  "gene": "UniProtKB:Q8N4C6",
  "gene_symbol": "NIN",
  "gene_name": "Ninein",
  "term_id": "GO:0051642"
}